{
  "term_label": "Unknown molecular function",
  "term_id": "UNKNOWN:0001",
  "gene": "UniProtKB:Q9P1G2",
  "gene_name": "Putative uncharacterized protein encoded by RBM12B-AS1",
  "gene_symbol": "RBM12B-AS1"
}